{
  "term_label": "transmembrane transporter activity",
  "gene": "UniProtKB:Q96ES6",
  "gene_name": "Major facilitator superfamily domain-containing protein 3",
  "gene_symbol": "MFSD3",
  "term_id": "GO:0022857"
}